cellular response to glial cell derived neurotrophic factor [GO:1990792] (BP) Also known as: cellular response to ATF, cellular response to GDNF, cellular response to astrocyte-derived trophic factor Relationships: is a type of cellular response to growth factor stimulus [GO:0071363]; is a type of response to glial cell derived neurotrophic factor [GO:1990790] Definition: Any process that results in a change in state or activity of a cell (in terms of movement, secretion, enzyme production, gene expression, etc.) as a result of a glial cell derived neurotrophic factor stimulus. References: PMID:20877310